{
  "term_id": "GO:0031012",
  "gene_name": "Serine protease HTRA1",
  "term_label": "extracellular matrix",
  "gene": "UniProtKB:Q92743",
  "gene_symbol": "HTRA1"
}